{
  "gene_symbol": "TRIP6",
  "gene": "UniProtKB:Q15654",
  "term_label": "cytoplasm",
  "term_id": "GO:0005737",
  "gene_name": "Thyroid receptor-interacting protein 6"
}